{
  "term_label": "THO complex part of transcription export complex",
  "gene": "UniProtKB:Q13769",
  "gene_name": "THO complex subunit 5 homolog",
  "term_id": "GO:0000445",
  "gene_symbol": "THOC5"
}